{
  "gene_name": "Transcription initiation factor TFIID subunit 1-like",
  "term_id": "GO:0051123",
  "gene": "UniProtKB:Q8IZX4",
  "gene_symbol": "TAF1L",
  "term_label": "RNA polymerase II preinitiation complex assembly"
}